sarcinapterin biosynthetic process [GO:1900868] (biological process) Definition: The chemical reactions and pathways resulting in the formation of sarcinapterin. Sources: GOC:TermGenie, GOC:mengo_curators Also known as: sarcinapterin anabolism, sarcinapterin biosynthesis, sarcinapterin formation, sarcinapterin synthesis Relationships: is a type of tricarboxylic acid biosynthetic process [GO:0072351]; is a type of sarcinapterin metabolic process [GO:1900867]; is a type of GO:2001116 Regulation: regulated by regulation of sarcinapterin biosynthetic process [GO:1900971]; negatively regulated by negative regulation of sarcinapterin biosynthetic process [GO:1900972]; positively regulated by GO:1900973